cell-cell fusion [GO:0140253] (biological process) Definition: A cellular process in which two or more cells combine together, their plasma membrane fusing, producing a single cell. In some cases, nuclei fuse, producing a polyploid cell, while in other cases, nuclei remain separate, producing a syncytium. Sources: Wikipedia:Cell_fusion Also known as: cell fusion, cell cell fusion Relationships: is a type of cellular process [GO:0009987]; has part GO:0045026 Subtypes: GO:0000768